{
  "gene_name": "Synaptotagmin-2",
  "gene": "UniProtKB:Q8N9I0",
  "term_id": "GO:0030672",
  "term_label": "synaptic vesicle membrane",
  "gene_symbol": "SYT2"
}